{
  "term_label": "Unknown cellular component",
  "term_id": "UNKNOWN:0003",
  "gene_symbol": "RASA4",
  "gene_name": "Ras GTPase-activating protein 4",
  "gene": "UniProtKB:O43374"
}